{
  "gene": "UniProtKB:P49638",
  "gene_symbol": "TTPA",
  "gene_name": "Alpha-tocopherol transfer protein",
  "term_id": "GO:0051180",
  "term_label": "vitamin transport"
}